glycosylphosphatidylinositol phospholipase D activity [GO:0004621] (molecular function) Sources: EC:3.1.4.50 Relationships: is a type of GO:0004630 Also known as: glycoprotein phospholipase D activity, GPI-PLD activity, glycoprotein-phosphatidylinositol phosphatidohydrolase activity, phosphatidylinositol phospholipase D activity, phosphatidylinositol-glycan-specific phospholipase D activity, phosphatidylinositol-specific phospholipase D activity Definition: Catalysis of the reaction: glycoprotein phosphatidylinositol + H2O = phosphatidate + glycoprotein inositol.